lysine-pyruvate 6-transaminase activity [GO:0050065] (molecular function) Relationships: is a type of GO:0008483 Note: Note that this term has a MetaCyc pathway reference as the pathway only has a single step. Also known as: lysine--pyruvate 6-aminotransferase activity, L-lysine:pyruvate aminotransferase activity, Lys-AT, lysine-pyruvate aminotransferase activity Definition: Catalysis of the reaction: L-lysine + pyruvate = L-alanine + L-allysine. Sources: EC:2.6.1.71, RHEA:19393